{
  "gene_name": "Glucose-fructose oxidoreductase domain-containing protein 1",
  "term_id": "UNKNOWN:0002",
  "gene": "UniProtKB:Q9NXC2",
  "term_label": "Unknown biological process",
  "gene_symbol": "GFOD1"
}